regulation of termination of RNA polymerase II transcription [GO:1904594] (biological process) References: PMID:25417108 Sources: GOC:TermGenie, GO_REF:0000058 Definition: Any process that modulates the frequency, rate or extent of termination of RNA polymerase II transcription. Also known as: regulation of RNA 3'-end formation by RNA polymerase II, regulation of RNA polymerase II transcription termination, regulation of transcription termination from Pol II promoter, regulation of transcription termination from RNA polymerase II promoter, regulation of RNA polymerase II transcription termination factor activity Subtypes: negative regulation of termination of RNA polymerase II transcription [GO:0120191], positive regulation of termination of RNA polymerase II transcription [GO:1904595], regulation of termination of RNA polymerase II transcription, poly(A)-coupled [GO:2000804] Relationships: is a type of regulation of termination of DNA-templated transcription [GO:0031554]; regulates GO:0006369